negative regulation of hepatocyte proliferation [GO:2000346] (biological process) Definition: Any process that stops, prevents or reduces the frequency, rate or extent of hepatocyte proliferation. Sources: GOC:BHF, GOC:mah Relationships: is a type of negative regulation of epithelial cell proliferation [GO:0050680]; is a type of regulation of hepatocyte proliferation [GO:2000345]; negatively regulates hepatocyte proliferation [GO:0072574]